{
  "term_id": "UNKNOWN:0002",
  "gene_name": "Collectin-10",
  "term_label": "Unknown biological process",
  "gene": "UniProtKB:Q9Y6Z7",
  "gene_symbol": "COLEC10"
}